{
  "term_id": "GO:0016514",
  "gene_symbol": "BICRA",
  "gene_name": "BRD4-interacting chromatin-remodeling complex-associated protein",
  "term_label": "SWI/SNF complex",
  "gene": "UniProtKB:Q9NZM4"
}